excitation of vasomotor center by aortic body chemoreceptor signaling [GO:0003040] (biological process) Relationships: is a type of excitation of vasomotor center by chemoreceptor signaling [GO:0002008]; is part of regulation of systemic arterial blood pressure by aortic body chemoreceptor signaling [GO:0003028] Also known as: excitation of vasomotor center by aortic body chemoreceptor signalling Sources: GOC:mtg_cardio Definition: The process in which the molecular signal from an aortic body is relayed to the vasomotor center, causing it to signal an increase arterial pressure.